{
  "term_label": "phospholipid binding",
  "gene": "UniProtKB:O95445",
  "gene_symbol": "APOM",
  "term_id": "GO:0005543",
  "gene_name": "Apolipoprotein M"
}